{
  "gene": "UniProtKB:Q14966",
  "term_label": "regulation of RNA splicing",
  "gene_name": "Zinc finger protein 638",
  "gene_symbol": "ZNF638",
  "term_id": "GO:0043484"
}